{
  "gene_name": "Carboxypeptidase A4",
  "term_id": "GO:0006508",
  "gene": "UniProtKB:Q9UI42",
  "term_label": "proteolysis",
  "gene_symbol": "CPA4"
}